{
  "term_id": "GO:0030032",
  "term_label": "lamellipodium assembly",
  "gene": "UniProtKB:O94929",
  "gene_symbol": "ABLIM3",
  "gene_name": "Actin-binding LIM protein 3"
}